{
  "term_label": "regulation of DNA-templated transcription",
  "gene_symbol": "RSF1",
  "gene": "UniProtKB:Q96T23",
  "term_id": "GO:0006355",
  "gene_name": "Remodeling and spacing factor 1"
}